peroxisome [GO:0005777] (cellular component) Definition: A small organelle enclosed by a single membrane, and found in most eukaryotic cells. Contains peroxidases and other enzymes involved in a variety of metabolic processes including free radical detoxification, lipid catabolism and biosynthesis, and hydrogen peroxide metabolism. References: PMID:9302272 Sources: GOC:pm, UniProtKB-KW:KW-0576 Also known as: peroxisome vesicle, peroxisomal Relationships: is a type of microbody [GO:0042579] Subtypes: GO:0009514, P1 peroxisome [GO:0019819], P2 peroxisome [GO:0019820], P3 peroxisome [GO:0019821], P4 peroxisome [GO:0019822], GO:0019823, P6 peroxisome [GO:0019824], glycosome [GO:0020015], mannosome [GO:0042580]